{
  "gene_name": "Myosin light chain 1_3, skeletal muscle isoform",
  "gene": "UniProtKB:P05976",
  "term_label": "microfilament motor activity",
  "term_id": "GO:0000146",
  "gene_symbol": "MYL1"
}